{
  "gene_name": "NHL-repeat-containing protein 4",
  "gene": "UniProtKB:P0CG21",
  "gene_symbol": "NHLRC4",
  "term_label": "Unknown cellular component",
  "term_id": "UNKNOWN:0003"
}